{
  "term_label": "regulation of cytokine production",
  "gene_name": "POZ-, AT hook-, and zinc finger-containing protein 1",
  "term_id": "GO:0001817",
  "gene_symbol": "PATZ1",
  "gene": "UniProtKB:Q9HBE1"
}